{
  "gene": "UniProtKB:O60882",
  "gene_symbol": "MMP20",
  "term_label": "amelogenesis",
  "gene_name": "Matrix metalloproteinase-20",
  "term_id": "GO:0097186"
}